{
  "gene_symbol": "RIMBP2",
  "term_id": "UNKNOWN:0001",
  "term_label": "Unknown molecular function",
  "gene_name": "RIMS-binding protein 2",
  "gene": "UniProtKB:O15034"
}